{
  "term_label": "nucleus",
  "term_id": "GO:0005634",
  "gene_name": "LIM_homeobox protein Lhx5",
  "gene": "UniProtKB:Q9H2C1",
  "gene_symbol": "LHX5"
}